{
  "term_label": "nucleus",
  "gene_symbol": "HSPA7",
  "term_id": "GO:0005634",
  "gene_name": "Putative heat shock 70 kDa protein 7",
  "gene": "UniProtKB:P48741"
}